{
  "gene_symbol": "BCAT2",
  "gene_name": "Branched-chain-amino-acid aminotransferase, mitochondrial",
  "gene": "UniProtKB:O15382",
  "term_label": "L-valine biosynthetic process",
  "term_id": "GO:0009099"
}